acyl-CoA (8-3)-desaturase activity [GO:0062076] (molecular function) Definition: Catalysis of the reaction: (8Z,11Z,14Z)-eicosatrienoyl-CoA + 2 Fe(II)-[cytochrome b5] + 2 H+ + O2 = (5Z,8Z,11Z,14Z)-eicosatetraenoyl-CoA + 2 Fe(III)-[cytochrome b5] + 2 H2O. Can also use a substrate with 3 double bonds (a (8Z,11Z,14Z,17Z)-eicosatetraenoyl-CoA) and add a fourth double bond (a (5Z,8Z,11Z,14Z,17Z)-eicosapentaenoyl-CoA). Relationships: is a type of acyl-CoA desaturase activity [GO:0016215] References: PMID:10601301, PMID:10769175 Sources: RHEA:46424 Also known as: acyl-CoA D5-desaturase activity, acyl-CoA delta(5)-desaturase activity, acyl-CoA delta5-desaturase activity